synapse assembly involved in innervation [GO:0060386] (BP) Relationships: is a type of synapse assembly [GO:0007416]; is part of GO:0060384 Also known as: synapse biogenesis involved in innervation, synaptogenesis involved in innervation Sources: GOC:dph, GOC:pr, GOC:sart Definition: The assembly of a synapse within a target tissue in which a nerve is invading.